{
  "term_id": "GO:0090042",
  "gene_symbol": "HDAC6",
  "gene": "UniProtKB:Q9UBN7",
  "term_label": "tubulin deacetylation",
  "gene_name": "Histone deacetylase 6"
}